{
  "term_id": "GO:0042781",
  "term_label": "3'-tRNA processing endoribonuclease activity",
  "gene_name": "Zinc phosphodiesterase ELAC protein 1",
  "gene": "UniProtKB:Q9H777",
  "gene_symbol": "ELAC1"
}